nucleobase-containing compound transmembrane transporter activity [GO:0015932] (molecular function) Relationships: is_a transmembrane transporter activity [GO:0022857]; BFO_0000050 nucleobase-containing compound transport [GO:0015931] Definition: Enables the transfer of nucleobases, nucleosides, nucleotides and nucleic acids from one side of a membrane to the other. Subtypes: nucleoside transmembrane transporter activity [GO:0005337], nucleotide-sugar transmembrane transporter activity [GO:0005338], nucleotide-sulfate transmembrane transporter activity [GO:0005340], GO:0008521, GO:0015215, GO:0015228, GO:0015607, nucleic acid transmembrane transporter activity [GO:0051032] Also known as: nucleobase, nucleoside, nucleotide and nucleic acid transmembrane transporter activity Sources: GOC:ai